{
  "gene_symbol": "NTF3",
  "term_id": "GO:0007169",
  "gene": "UniProtKB:P20783",
  "gene_name": "Neurotrophin-3",
  "term_label": "cell surface receptor protein tyrosine kinase signaling pathway"
}